heterotrimeric G-protein complex [GO:0005834] (CC) Note: See also the molecular function term 'G protein-coupled receptor activity ; GO:0004930'. Also known as: heterotrimeric G-protein GTPase, alpha-subunit, heterotrimeric G-protein GTPase, beta-subunit, heterotrimeric G-protein GTPase, gamma-subunit, heterotrimeric G-protein GTPase activity Definition: Any of a family of heterotrimeric GTP-binding and hydrolyzing proteins; they belong to a superfamily of GTPases that includes monomeric proteins such as EF-Tu and RAS. Heterotrimeric G-proteins consist of three subunits; the alpha subunit contains the guanine nucleotide binding site and possesses GTPase activity; the beta and gamma subunits are tightly associated and function as a beta-gamma heterodimer; extrinsic plasma membrane proteins (cytoplasmic face) that function as a complex to transduce signals from G protein-coupled receptors to an effector protein. Relationships: is a type of plasma membrane protein complex [GO:0098797]; is a type of GO:1905360; is part of extrinsic component of cytoplasmic side of plasma membrane [GO:0031234] Sources: ISBN:0198547684